{
  "gene_name": "CDAN1-interacting nuclease 1",
  "gene": "UniProtKB:Q9Y2V0",
  "term_label": "Unknown molecular function",
  "term_id": "UNKNOWN:0001",
  "gene_symbol": "CDIN1"
}